{
  "gene_symbol": "TRBV9",
  "term_id": "UNKNOWN:0001",
  "gene": "UniProtKB:A0A0B4J1U6",
  "gene_name": "T cell receptor beta variable 9",
  "term_label": "Unknown molecular function"
}